{
  "term_label": "Unknown biological process",
  "gene_symbol": "PWWP4",
  "gene": "UniProtKB:A0A494C071",
  "gene_name": "PWWP domain-containing DNA repair factor 4",
  "term_id": "UNKNOWN:0002"
}